{
  "gene": "UniProtKB:P17948",
  "gene_name": "Vascular endothelial growth factor receptor 1",
  "gene_symbol": "FLT1",
  "term_label": "cell migration",
  "term_id": "GO:0016477"
}